regulation of twitch skeletal muscle contraction [GO:0014724] (biological process) Sources: GOC:mtg_muscle Relationships: is a type of regulation of skeletal muscle contraction [GO:0014819]; regulates twitch skeletal muscle contraction [GO:0014721] Definition: Any process that modulates the frequency, rate or extent of twitch skeletal muscle contraction. Subtypes: regulation of fast-twitch skeletal muscle fiber contraction [GO:0031446], regulation of slow-twitch skeletal muscle fiber contraction [GO:0031449]